regulation of synaptic vesicle transport [GO:1902803] (biological process) Also known as: regulation of synaptic vesicle fission, regulation of synaptic vesicle fusion Subtypes: negative regulation of synaptic vesicle transport [GO:1902804], positive regulation of synaptic vesicle transport [GO:1902805], regulation of anterograde synaptic vesicle transport [GO:1903742] References: PMID:23527112 Sources: GOC:TermGenie, GOC:kmv, GO_REF:0000058 Definition: Any process that modulates the frequency, rate or extent of synaptic vesicle transport. Relationships: is a type of regulation of cellular process [GO:0050794]; is a type of regulation of transport [GO:0051049]; regulates GO:0048489